ascus membrane [GO:0036362] (cellular component) References: PMID:21900489 Sources: GOC:mcc, GOC:vw Definition: A double layer of lipid molecules that surrounds an ascus, a capsule containing the sexual spores in some fungi. Relationships: is a type of membrane [GO:0016020]